{
  "gene": "UniProtKB:Q96RI9",
  "gene_name": "Trace amine-associated receptor 9",
  "gene_symbol": "TAAR9",
  "term_id": "GO:0001594",
  "term_label": "trace-amine receptor activity"
}